{
  "gene_symbol": "CLDN4",
  "gene_name": "Claudin-4",
  "term_label": "renal absorption",
  "term_id": "GO:0070293",
  "gene": "UniProtKB:O14493"
}